{
  "term_id": "GO:0005886",
  "gene_name": "Phosphatidylcholine:ceramide cholinephosphotransferase 2",
  "gene_symbol": "SGMS2",
  "gene": "UniProtKB:Q8NHU3",
  "term_label": "plasma membrane"
}